eIF2alpha dephosphorylation in response to endoplasmic reticulum stress [GO:0036497] (biological process) Relationships: is a type of regulation of translation initiation in response to endoplasmic reticulum stress [GO:0036491]; is a type of regulation of translational initiation by eIF2 alpha dephosphorylation [GO:0036496] Definition: The removal of a phosphate group from the translation initiation factor eIF2alpha, as a result of endoplasmic reticulum stress. References: PMID:16835242 Sources: GOC:PARL, GOC:bf Also known as: eIF2alpha dephosphorylation in response to ER stress, regulation of translation initiation by eIF2alpha dephosphorylation in response to endoplasmic reticulum stress